{
  "gene": "UniProtKB:P01871",
  "gene_symbol": "IGHM",
  "term_label": "Unknown cellular component",
  "gene_name": "Immunoglobulin heavy constant mu",
  "term_id": "UNKNOWN:0003"
}